histone H2AT120 kinase activity [GO:1990244] (molecular function) Also known as: histone H2A-T120 kinase activity, histone H2AS120 kinase activity, histone kinase activity (H2A-T120 specific), histone threonine kinase activity (H2A-T120 specific) References: PMID:24140421 Definition: Catalysis of the reaction: histone H2A-threonine (position 120) + ATP = histone H2A-phosphothreonine (position 120) + ADP. This reaction is the addition of a phosphate group to the threonine residue at position 120 of histone H2A. Relationships: is a type of protein serine/threonine kinase activity [GO:0004674]; is a type of GO:0140995 Note: Note that the residue position corresponds to the canonical human H2A2A histone (UniProtKB:Q6FI13); this residue is conserved across all eukaryotes, but corresponds to T119 in Drosophila and S121 in yeast and Tetrahymena. Residue 1 is the first residue following removal of the initiating Methionine (Met). Note that each histone is encoded by multiple genes, and sequences may vary across different genes within an organism.